{
  "term_label": "Unknown cellular component",
  "gene_symbol": "PCYT1B",
  "gene": "UniProtKB:Q9Y5K3",
  "gene_name": "Choline-phosphate cytidylyltransferase B",
  "term_id": "UNKNOWN:0003"
}